regulation of small molecule metabolic process [GO:0062012] (biological process) Sources: GOC:vw Subtypes: GO:0006140, regulation of purine nucleobase metabolic process [GO:0006141], GO:0009118, regulation of salicylic acid metabolic process [GO:0010337], GO:0010371, GO:0010439, regulation of ketone biosynthetic process [GO:0010566], regulation of ketone catabolic process [GO:0010567], regulation of 1-aminocyclopropane-1-carboxylate metabolic process [GO:0010602], regulation of glucose metabolic process [GO:0010906], GO:0019217, regulation of vitamin metabolic process [GO:0030656], regulation of aldosterone metabolic process [GO:0032344], regulation of penicillin catabolic process [GO:0033247], regulation of urea catabolic process [GO:0034254], GO:0043463, regulation of fucose catabolic process [GO:0043468], regulation of D-xylose catabolic process [GO:0043469], GO:0045734, positive regulation of small molecule metabolic process [GO:0062013], negative regulation of small molecule metabolic process [GO:0062014], regulation of taurine biosynthetic process [GO:0062089], regulation of L-glutamine biosynthetic process [GO:0062132], GO:0070857, GO:0080020, GO:0090181, regulation of nitrate assimilation [GO:0090352], regulation of L-tryptophan metabolic process [GO:0090357], regulation of ornithine metabolic process [GO:0090368], regulation of (R)-mevalonic acid biosynthetic process [GO:0106107], regulation of UDP-N-acetylglucosamine biosynthetic process [GO:0106278], regulation of histidine biosynthetic process [GO:0120213], regulation of arginine biosynthetic process [GO:1900079], regulation of arginine catabolic process [GO:1900081], regulation of aflatoxin biosynthetic process [GO:1900177], regulation of penicillin biosynthetic process [GO:1900196], regulation of methane biosynthetic process from formic acid [GO:1900339], regulation of alcohol catabolic process [GO:1900419], regulation of emericellamide biosynthetic process [GO:1900658], regulation of fumonisin biosynthetic process [GO:1900683], GO:1900686, regulation of o-orsellinic acid biosynthetic process [GO:1900698], regulation of pseurotin A biosynthetic process [GO:1900849], regulation of sarcinapterin biosynthetic process [GO:1900971], regulation of tatiopterin biosynthetic process [GO:1900974], GO:1901413, GO:1901466, regulation of cysteine metabolic process [GO:1901494], regulation of homoserine biosynthetic process [GO:1901710], GO:1901715, regulation of fumagillin biosynthetic process [GO:1902090], regulation of alcohol biosynthetic process [GO:1902930], regulation of lysine biosynthetic process via aminoadipic acid [GO:1902986], regulation of L-dopa biosynthetic process [GO:1903195], regulation of citrulline biosynthetic process [GO:1903248], GO:1904984, regulation of glutamate metabolic process [GO:2000211], regulation of L-proline metabolic process [GO:2000214], regulation of glyoxylate cycle [GO:2000874], GO:2001154, regulation of isopentenyl diphosphate biosynthetic process, mevalonate pathway [GO:2001210], regulation of L-leucine biosynthetic process [GO:2001276] Relationships: is a type of regulation of metabolic process [GO:0019222]; regulates GO:0044281 Also known as: regulation of small molecule metabolism Definition: Any process that modulates the rate, frequency or extent of a small molecule metabolic process.